{
  "gene_name": "Cytochrome P450 2A13",
  "term_id": "GO:0009804",
  "gene": "UniProtKB:Q16696",
  "term_label": "coumarin metabolic process",
  "gene_symbol": "CYP2A13"
}